{
  "term_label": "Unknown molecular function",
  "gene": "UniProtKB:A0A075B6X5",
  "gene_name": "T cell receptor alpha variable 18",
  "term_id": "UNKNOWN:0001",
  "gene_symbol": "TRAV18"
}